{
  "gene_name": "Peroxisome proliferator-activated receptor gamma",
  "gene_symbol": "PPARG",
  "term_id": "GO:0030154",
  "term_label": "cell differentiation",
  "gene": "UniProtKB:P37231"
}